positive regulation of apical constriction involved in ventral furrow formation [GO:0110074] (biological process) Definition: Any process that activates or increases the frequency, rate or extent of apical constriction involved in ventral furrow formation. Relationships: is a type of regulation of apical constriction involved in ventral furrow formation [GO:0110073]; is a type of positive regulation of actin filament-based movement [GO:1903116]; positively regulates GO:0110072 References: PMID:28495958 Sources: GOC:ha